{
  "term_id": "UNKNOWN:0001",
  "gene_symbol": "SEPTIN14P20",
  "term_label": "Unknown molecular function",
  "gene_name": "Putative RNA-binding regulatory peptide",
  "gene": "UniProtKB:C0HM01"
}